{
  "term_label": "oligosaccharide binding",
  "term_id": "GO:0070492",
  "gene_symbol": "SELL",
  "gene_name": "L-selectin",
  "gene": "UniProtKB:P14151"
}